Bfa1-Bub2 complex [GO:1990334] (cellular component) Definition: A protein complex that acts as a two-component GTPase-activating protein for Tem1 GTPase, thus regulating a signal transduction cascade, called the mitotic exit network (MEN), which is required for mitotic exit and cytokinesis. Bub2/Bfa1 keeps Tem1 inactive until the spindle is properly oriented, thus inhibiting MEN activation. References: PMID:16449187 Sources: GOC:bhm Relationships: is a type of GTPase activator complex [GO:1902773]; is part of spindle pole body [GO:0005816]